DNA replication initiation [GO:0006270] (biological process) Regulation: regulated by regulation of DNA-templated DNA replication initiation [GO:0030174]; negatively regulated by GO:0032297; positively regulated by positive regulation of DNA-templated DNA replication initiation [GO:0032298] Relationships: is_a DNA metabolic process [GO:0006259]; is part of DNA-templated DNA replication [GO:0006261] Subtypes: cell cycle DNA replication initiation [GO:1902292] Also known as: DNA-dependent DNA replication initiation, DNA endoreduplication initiation, DNA re-replication initiation Definition: The process in which DNA-dependent DNA replication is started; it begins when specific sequences, known as origins of replication, are recognized and bound by the origin recognition complex, followed by DNA unwinding. References: PMID:28209641